{
  "term_id": "UNKNOWN:0002",
  "gene_symbol": "IRF2BPL",
  "gene": "UniProtKB:Q9H1B7",
  "gene_name": "Probable E3 ubiquitin-protein ligase IRF2BPL",
  "term_label": "Unknown biological process"
}